{
  "gene_symbol": "LCN9",
  "term_id": "UNKNOWN:0001",
  "gene": "UniProtKB:Q8WX39",
  "term_label": "Unknown molecular function",
  "gene_name": "Epididymal-specific lipocalin-9"
}